negative regulation of regulatory T cell differentiation [GO:0045590] (BP) Definition: Any process that stops, prevents, or reduces the rate of differentiation of regulatory T cells. Note: Note that immunologists typically use the word 'development' to refer to cells of B or T cell lineages undergoing the process that GO describes as 'cell differentiation'. Sources: ISBN:0781735149 Subtypes: negative regulation of CD4-positive, CD25-positive, alpha-beta regulatory T cell differentiation [GO:0032830] Relationships: is a type of negative regulation of T cell differentiation [GO:0045581]; is a type of regulation of regulatory T cell differentiation [GO:0045589]; negatively regulates regulatory T cell differentiation [GO:0045066] Also known as: down regulation of regulatory T cell differentiation, down-regulation of regulatory T cell differentiation, downregulation of regulatory T cell differentiation, negative regulation of regulatory T lymphocyte differentiation, negative regulation of regulatory T-cell differentiation, negative regulation of regulatory T-lymphocyte differentiation, negative regulation of suppressor T cell differentiation, negative regulation of suppressor T-cell differentiation, inhibition of regulatory T cell differentiation, negative regulation of regulatory T cell development